{
  "gene_symbol": "HEXIM2",
  "gene_name": "Protein HEXIM2",
  "term_label": "cytoplasm",
  "gene": "UniProtKB:Q96MH2",
  "term_id": "GO:0005737"
}